{
  "gene": "UniProtKB:Q6VB84",
  "gene_name": "Forkhead box protein D4-like 3",
  "term_label": "cell differentiation",
  "term_id": "GO:0030154",
  "gene_symbol": "FOXD4L3"
}